L-methionine salvage from S-adenosylmethionine [GO:0019284] (biological process) Definition: The chemical reactions and pathways resulting in the formation of L-methionine from S-adenosylmethionine. Relationships: is a type of L-methionine salvage [GO:0071267]; is part of S-adenosylmethionine cycle [GO:0033353] Also known as: L-methionine formation from S-adenosylmethionine, L-methionine synthesis from S-adenosylmethionine References: PMID:31950558 Sources: GOC:go_curators, GOC:vw